{
  "term_id": "GO:0004674",
  "gene": "UniProtKB:P53667",
  "term_label": "protein serine/threonine kinase activity",
  "gene_name": "LIM domain kinase 1",
  "gene_symbol": "LIMK1"
}